{
  "term_id": "GO:0005783",
  "gene": "UniProtKB:Q9BRK5",
  "term_label": "endoplasmic reticulum",
  "gene_symbol": "SDF4",
  "gene_name": "45 kDa calcium-binding protein"
}